{
  "gene_symbol": "PTMS",
  "term_label": "positive regulation of transcription by RNA polymerase II",
  "gene_name": "Parathymosin",
  "gene": "UniProtKB:P20962",
  "term_id": "GO:0045944"
}